{
  "term_id": "GO:0005886",
  "gene": "UniProtKB:Q15049",
  "term_label": "plasma membrane",
  "gene_symbol": "MLC1",
  "gene_name": "Membrane protein MLC1"
}